{
  "term_label": "Unknown cellular component",
  "term_id": "UNKNOWN:0003",
  "gene_name": "FXYD domain-containing ion transport regulator 3",
  "gene": "UniProtKB:Q14802",
  "gene_symbol": "FXYD3"
}